{
  "term_label": "lumenal side of endoplasmic reticulum membrane",
  "gene_name": "Signal peptide peptidase-like 2B",
  "gene": "UniProtKB:Q8TCT7",
  "term_id": "GO:0098553",
  "gene_symbol": "SPPL2B"
}